{
  "gene": "UniProtKB:O14581",
  "gene_symbol": "OR7A17",
  "term_id": "GO:0005886",
  "gene_name": "Olfactory receptor 7A17",
  "term_label": "plasma membrane"
}